{
  "gene_name": "Ras guanyl-releasing protein 3",
  "term_id": "GO:0005886",
  "gene": "UniProtKB:Q8IV61",
  "term_label": "plasma membrane",
  "gene_symbol": "RASGRP3"
}